{
  "term_id": "GO:0006366",
  "term_label": "transcription by RNA polymerase II",
  "gene_name": "Transcription initiation factor IIA subunit 1",
  "gene": "UniProtKB:P52655",
  "gene_symbol": "GTF2A1"
}